{
  "gene_symbol": "DCTN1",
  "gene_name": "Dynactin subunit 1",
  "gene": "UniProtKB:Q14203",
  "term_label": "axon",
  "term_id": "GO:0030424"
}